ISG15-specific peptidase activity [GO:0019785] (molecular function) Definition: A thiol-dependent isopeptidase activity that cleaves ISG15 from a target protein to which it is conjugated. References: PMID:30213559 Sources: GOC:mah Also known as: ISG15-specific protease activity Relationships: is a type of cysteine-type peptidase activity [GO:0008234]; is a type of ubiquitin-like protein peptidase activity [GO:0019783]